bacterial-type flagellum-dependent swimming motility [GO:0071977] (biological process) Definition: Bacterial-type flagellum-dependent cell motility that results in the smooth movement of a cell through a liquid medium. References: PMID:18461074 Sources: GOC:cilia Also known as: bacterial-type flagellum-mediated cell swimming, bacterial-type flagellar swimming motility Relationships: is a type of bacterial-type flagellum-dependent cell motility [GO:0071973]; is a type of cell swimming [GO:0071975]